{
  "gene_name": "C-C motif chemokine 5",
  "term_label": "chemokine-mediated signaling pathway",
  "gene": "UniProtKB:P13501",
  "gene_symbol": "CCL5",
  "term_id": "GO:0070098"
}